{
  "gene_symbol": "ESM1",
  "term_id": "GO:1902204",
  "gene_name": "Endothelial cell-specific molecule 1",
  "term_label": "positive regulation of hepatocyte growth factor receptor signaling pathway",
  "gene": "UniProtKB:Q9NQ30"
}